{
  "gene_symbol": "NOTCH2NLB",
  "term_id": "UNKNOWN:0002",
  "gene_name": "Notch homolog 2 N-terminal-like protein B",
  "term_label": "Unknown biological process",
  "gene": "UniProtKB:P0DPK3"
}